{
  "gene_name": "PACRG-like protein",
  "gene": "UniProtKB:Q8N7B6",
  "term_label": "Unknown biological process",
  "term_id": "UNKNOWN:0002",
  "gene_symbol": "PACRGL"
}